lamellar body [GO:0042599] (cellular component) Definition: A membrane-bounded organelle, specialized for the storage and secretion of various substances (surfactant phospholipids, glycoproteins and acid phosphates) which are arranged in the form of tightly packed, concentric, membrane sheets or lamellae. Has some similar properties to, but is distinct from, a lysosome. Also known as: lamellar granule, membrane-coating granule, Odland body, keratinosome Subtypes: alveolar lamellar body [GO:0097208], epidermal lamellar body [GO:0097209], dendritic lamellar body [GO:1990503] References: PMID:12243725 Sources: GOC:cjm, GOC:jl, Wikipedia:Lamellar_granule Relationships: is a type of GO:0030141